{
  "term_label": "Unknown molecular function",
  "gene": "UniProtKB:O75354",
  "term_id": "UNKNOWN:0001",
  "gene_symbol": "ENTPD6",
  "gene_name": "Ectonucleoside triphosphate diphosphohydrolase 6"
}